{
  "term_label": "chromatin remodeling",
  "gene_name": "Lysine-specific demethylase 4D",
  "gene": "UniProtKB:Q6B0I6",
  "gene_symbol": "KDM4D",
  "term_id": "GO:0006338"
}